{
  "term_id": "GO:0005737",
  "gene": "UniProtKB:Q5T5C0",
  "term_label": "cytoplasm",
  "gene_symbol": "STXBP5",
  "gene_name": "Syntaxin-binding protein 5"
}